{
  "gene_symbol": "PIK3CG",
  "term_label": "phosphatidylinositol 3-kinase complex, class IB",
  "gene_name": "Phosphatidylinositol 4,5-bisphosphate 3-kinase catalytic subunit gamma isoform",
  "gene": "UniProtKB:P48736",
  "term_id": "GO:0005944"
}